{
  "gene_name": "Olfactory receptor 8H3",
  "gene": "UniProtKB:Q8N146",
  "term_label": "olfactory receptor activity",
  "gene_symbol": "OR8H3",
  "term_id": "GO:0004984"
}